{
  "term_id": "UNKNOWN:0003",
  "term_label": "Unknown cellular component",
  "gene_name": "Histone-lysine N-methyltransferase PRDM7",
  "gene_symbol": "PRDM7",
  "gene": "UniProtKB:Q9NQW5"
}